{
  "gene": "UniProtKB:Q7Z7J9",
  "gene_symbol": "CAMK2N1",
  "gene_name": "Calcium_calmodulin-dependent protein kinase II inhibitor 1",
  "term_label": "Unknown biological process",
  "term_id": "UNKNOWN:0002"
}